{
  "term_id": "GO:0048020",
  "gene_symbol": "CCL26",
  "term_label": "CCR chemokine receptor binding",
  "gene_name": "C-C motif chemokine 26",
  "gene": "UniProtKB:Q9Y258"
}